Rb-E2F complex [GO:0035189] (cellular component) Relationships: is a type of RNA polymerase II transcription regulator complex [GO:0090575] Definition: A multiprotein complex containing a heterodimeric E2F transcription factor and a Retinoblastoma (Rb) family member. This complex is capable of repressing transcription of E2F-regulated genes in order to regulate cell cycle progression. Also known as: retinoblastoma-E2F complex References: PMID:14616073